{
  "gene_name": "Mast_stem cell growth factor receptor Kit",
  "term_id": "GO:0046427",
  "gene": "UniProtKB:P10721",
  "term_label": "positive regulation of receptor signaling pathway via JAK-STAT",
  "gene_symbol": "KIT"
}